fasciculation of motor neuron axon [GO:0097156] (biological process) Relationships: is a type of axonal fasciculation [GO:0007413] References: PMID:18403711 Sources: GOC:lb Definition: The collection of motor neuron axons into a bundle of rods, known as a fascicle.